negative regulation of oogenesis [GO:1905880] (biological process) Also known as: down regulation of oogenesis, down regulation of ovum development, down-regulation of oogenesis, down-regulation of ovum development, downregulation of oogenesis, downregulation of ovum development, negative regulation of ovum development, inhibition of oogenesis, inhibition of ovum development References: PMID:26434723 Sources: GOC:TermGenie, GO_REF:0000058 Relationships: is a type of GO:0010721; is a type of negative regulation of multicellular organismal process [GO:0051241]; is a type of regulation of oogenesis [GO:1905879]; is a type of negative regulation of reproductive process [GO:2000242]; negatively regulates oogenesis [GO:0048477] Definition: Any process that stops, prevents or reduces the frequency, rate or extent of oogenesis.